{
  "gene_symbol": "SP4",
  "term_label": "RNA polymerase II cis-regulatory region sequence-specific DNA binding",
  "gene_name": "Transcription factor Sp4",
  "gene": "UniProtKB:Q02446",
  "term_id": "GO:0000978"
}